clathrin-mediated membrane bending [GO:0097754] (biological process) Sources: GOC:pr, Wikipedia:Membrane_curvature Relationships: is a type of membrane bending [GO:0097753]; has part clathrin coat assembly [GO:0048268] Definition: A membrane bending process mediated by clathrin.